{
  "gene": "UniProtKB:Q96JY6",
  "gene_symbol": "PDLIM2",
  "term_id": "GO:0007507",
  "gene_name": "PDZ and LIM domain protein 2",
  "term_label": "heart development"
}